extrinsic component of membrane [GO:0019898] (cellular component) Definition: The component of a membrane consisting of gene products and protein complexes that are loosely bound to one of its surfaces, but not integrated into the hydrophobic region. Relationships: is a type of cellular anatomical structure [GO:0110165]; is part of GO:0016020 Note: Note that proteins extrinsic to membranes can be removed by treatments that do not disrupt the membrane, such as salt solutions. Sources: GOC:dos, GOC:jl, GOC:mah Subtypes: extrinsic component of plasma membrane [GO:0019897], extrinsic component of cell outer membrane [GO:0031244], extrinsic component of organelle membrane [GO:0031312], extrinsic component of thylakoid membrane [GO:0035448] Also known as: extrinsic to membrane, peripheral membrane protein